{
  "gene_symbol": "PDE6H",
  "gene": "UniProtKB:Q13956",
  "gene_name": "Retinal cone rhodopsin-sensitive cGMP 3',5'-cyclic phosphodiesterase subunit gamma",
  "term_label": "photoreceptor outer segment membrane",
  "term_id": "GO:0042622"
}